{
  "gene_name": "U6 snRNA-associated Sm-like protein LSm6",
  "gene": "UniProtKB:P62312",
  "term_label": "nucleolus",
  "term_id": "GO:0005730",
  "gene_symbol": "LSM6"
}